{
  "gene": "UniProtKB:Q7L5Y9",
  "term_label": "GID complex",
  "gene_name": "E3 ubiquitin-protein transferase MAEA",
  "term_id": "GO:0034657",
  "gene_symbol": "MAEA"
}